{
  "gene_symbol": "PATE1",
  "gene": "UniProtKB:Q8WXA2",
  "term_label": "Unknown cellular component",
  "term_id": "UNKNOWN:0003",
  "gene_name": "Prostate and testis expressed protein 1"
}